{
  "term_label": "nucleus",
  "gene_name": "Probable global transcription activator SNF2L2",
  "term_id": "GO:0005634",
  "gene": "UniProtKB:P51531",
  "gene_symbol": "SMARCA2"
}